{
  "gene_symbol": "CPLX3",
  "gene": "UniProtKB:Q8WVH0",
  "term_id": "GO:0031630",
  "gene_name": "Complexin-3",
  "term_label": "regulation of synaptic vesicle fusion to presynaptic active zone membrane"
}